 [license]